{
  "gene_name": "Hepatic leukemia factor",
  "term_label": "positive regulation of transcription by RNA polymerase II",
  "term_id": "GO:0045944",
  "gene": "UniProtKB:Q16534",
  "gene_symbol": "HLF"
}